{
  "gene_symbol": "OR2T33",
  "gene": "UniProtKB:Q8NG76",
  "term_label": "olfactory receptor activity",
  "gene_name": "Olfactory receptor 2T33",
  "term_id": "GO:0004984"
}